{
  "term_label": "positive regulation of macrophage fusion",
  "gene": "UniProtKB:O43914",
  "term_id": "GO:0034241",
  "gene_symbol": "TYROBP",
  "gene_name": "TYRO protein tyrosine kinase-binding protein"
}